positive regulation of cytotoxic T cell differentiation [GO:0045585] (BP) Relationships: is_a positive regulation of T cell differentiation [GO:0045582]; is a type of regulation of cytotoxic T cell differentiation [GO:0045583]; positively regulates GO:0045065 Sources: GOC:go_curators Also known as: positive regulation of cytotoxic T lymphocyte differentiation, positive regulation of cytotoxic T-cell differentiation, positive regulation of cytotoxic T-lymphocyte differentiation, up regulation of cytotoxic T cell differentiation, up-regulation of cytotoxic T cell differentiation, upregulation of cytotoxic T cell differentiation, activation of cytotoxic T cell differentiation, stimulation of cytotoxic T cell differentiation, positive regulation of cytotoxic T cell development Definition: Any process that activates or increases the frequency, rate or extent of cytotoxic T cell differentiation. Note: Note that immunologists typically use the word 'development' to refer to cells of B or T cell lineages undergoing the process that GO describes as 'cell differentiation'.